{
  "term_id": "GO:0005737",
  "gene_name": "Filensin",
  "gene": "UniProtKB:Q12934",
  "gene_symbol": "BFSP1",
  "term_label": "cytoplasm"
}